{
  "term_id": "GO:0097225",
  "gene_name": "Androglobin",
  "gene_symbol": "ADGB",
  "gene": "UniProtKB:Q8N7X0",
  "term_label": "sperm midpiece"
}